{
  "gene_name": "Homeobox protein NANOG",
  "term_id": "GO:0019827",
  "gene": "UniProtKB:Q9H9S0",
  "term_label": "stem cell population maintenance",
  "gene_symbol": "NANOG"
}